{
  "term_id": "UNKNOWN:0003",
  "gene_symbol": "BANP",
  "gene_name": "Protein BANP",
  "gene": "UniProtKB:Q8N9N5",
  "term_label": "Unknown cellular component"
}